{
  "term_id": "GO:0007160",
  "gene": "UniProtKB:Q14112",
  "gene_symbol": "NID2",
  "gene_name": "Nidogen-2",
  "term_label": "cell-matrix adhesion"
}